{
  "gene_name": "Gamma-synuclein",
  "gene_symbol": "SNCG",
  "term_label": "cytoplasm",
  "term_id": "GO:0005737",
  "gene": "UniProtKB:O76070"
}